flurbiprofen binding [GO:0035923] (molecular function) Also known as: 2-(2-fluoro-[1,1'-biphenyl-4-yl])propanoic acid binding Relationships: is a type of GO:0031406 Definition: Binding to flurbiprofen. Sources: GOC:BHF, GOC:rl